basal pole of outer hair cell [GO:0090712] (cellular component) References: PMID:12845523 Sources: GOC:sl Relationships: is a type of cell pole [GO:0060187] Definition: The end of the outer hair cell which receives and transmits neural signals.